{
  "term_label": "extracellular space",
  "gene_name": "Interferon alpha-21",
  "term_id": "GO:0005615",
  "gene_symbol": "IFNA21",
  "gene": "UniProtKB:P01568"
}